{
  "gene": "UniProtKB:P45378",
  "term_id": "GO:0005523",
  "term_label": "tropomyosin binding",
  "gene_name": "Troponin T, fast skeletal muscle",
  "gene_symbol": "TNNT3"
}